positive regulation of growth hormone secretion [GO:0060124] (BP) Definition: Any process that increases the frequency, rate or extent of the regulated release of growth hormone from a cell. Sources: GOC:dph Relationships: is a type of regulation of growth hormone secretion [GO:0060123]; is a type of positive regulation of peptide hormone secretion [GO:0090277]; positively regulates GO:0030252